negative regulation of transcription elongation by RNA polymerase II [GO:0034244] (biological process) Relationships: is a type of negative regulation of DNA-templated transcription, elongation [GO:0032785]; is a type of regulation of transcription elongation by RNA polymerase II [GO:0034243]; negatively regulates transcription elongation by RNA polymerase II [GO:0006368] Also known as: negative regulation of RNA elongation from RNA polymerase II promoter, negative regulation of transcription elongation from RNA polymerase II promoter, negative regulation of gene-specific transcription elongation from RNA polymerase II promoter Sources: GOC:mah, GOC:txnOH Definition: Any process that stops, prevents, or reduces the frequency, rate or extent of transcription elongation, the extension of an RNA molecule after transcription initiation and promoter clearance by the addition of ribonucleotides, catalyzed by RNA polymerase II.